axonogenesis involved in innervation [GO:0060385] (biological process) Sources: GOC:dph, GOC:sart Relationships: is a type of axonogenesis [GO:0007409]; is part of innervation [GO:0060384] Definition: The neurite development process that generates a long process of a neuron, as it invades a target tissue.